alpha-aminoacyl-tRNA binding [GO:1904678] (molecular function) Sources: GOC:TermGenie, GO_REF:0000067, ISBN:155581073X Definition: Binding to an alpha-aminoacyl-tRNA. Relationships: is a type of RNA binding [GO:0003723] Also known as: aminoacyl-tRNA binding